{
  "term_id": "GO:0005102",
  "gene_name": "Na(+)_H(+) exchange regulatory cofactor NHE-RF3",
  "gene_symbol": "PDZK1",
  "gene": "UniProtKB:Q5T2W1",
  "term_label": "signaling receptor binding"
}